{
  "gene": "UniProtKB:Q96CD0",
  "term_label": "SCF ubiquitin ligase complex",
  "gene_name": "F-box_LRR-repeat protein 8",
  "term_id": "GO:0019005",
  "gene_symbol": "FBXL8"
}